{
  "gene_symbol": "MYPN",
  "gene": "UniProtKB:Q86TC9",
  "term_id": "GO:0070593",
  "term_label": "dendrite self-avoidance",
  "gene_name": "Myopalladin"
}